{
  "term_id": "GO:0005085",
  "gene_name": "Rho guanine nucleotide exchange factor 16",
  "gene_symbol": "ARHGEF16",
  "gene": "UniProtKB:Q5VV41",
  "term_label": "guanyl-nucleotide exchange factor activity"
}